{
  "gene_symbol": "OR52E1",
  "term_id": "GO:0004984",
  "gene": "UniProtKB:Q8NGJ3",
  "term_label": "olfactory receptor activity",
  "gene_name": "Olfactory receptor 52E1"
}